{
  "gene_name": "COP9 signalosome complex subunit 8",
  "term_label": "COP9 signalosome",
  "term_id": "GO:0008180",
  "gene_symbol": "COPS8",
  "gene": "UniProtKB:Q99627"
}